{
  "gene": "UniProtKB:P48357",
  "term_id": "GO:0009897",
  "term_label": "external side of plasma membrane",
  "gene_symbol": "LEPR",
  "gene_name": "Leptin receptor"
}